{
  "gene": "UniProtKB:Q6ZNA4",
  "gene_name": "E3 ubiquitin-protein ligase Arkadia",
  "term_id": "GO:0006511",
  "term_label": "ubiquitin-dependent protein catabolic process",
  "gene_symbol": "RNF111"
}